positive regulation of Schwann cell differentiation [GO:0014040] (biological process) Also known as: up regulation of Schwann cell differentiation, up-regulation of Schwann cell differentiation, upregulation of Schwann cell differentiation, activation of Schwann cell differentiation, stimulation of Schwann cell differentiation Sources: GOC:ef Definition: Any process that activates or increases the frequency, rate or extent of Schwann cell differentiation. Relationships: is a type of regulation of Schwann cell differentiation [GO:0014038]; is_a positive regulation of glial cell differentiation [GO:0045687]; positively regulates GO:0014037